{
  "gene": "UniProtKB:Q14565",
  "gene_symbol": "DMC1",
  "term_label": "ATP-dependent activity, acting on DNA",
  "gene_name": "Meiotic recombination protein DMC1_LIM15 homolog",
  "term_id": "GO:0008094"
}